intrinsic apoptotic signaling pathway in response to osmotic stress [GO:0008627] (biological process) References: PMID:11454444, PMID:16483738 Sources: GOC:mtg_apoptosis Subtypes: intrinsic apoptotic signaling pathway in response to osmotic stress by p53 class mediator [GO:1990127] Relationships: is a type of GO:0071470; is a type of GO:0097193 Definition: The series of molecular signals in which an intracellular signal is conveyed to trigger the apoptotic death of a cell. The pathway is induced in response to changes in intracellular ion homeostasis, and ends when the execution phase of apoptosis is triggered. Also known as: induction of apoptosis by ionic changes Regulation: regulated by regulation of intrinsic apoptotic signaling pathway in response to osmotic stress [GO:1902218]; negatively regulated by negative regulation of intrinsic apoptotic signaling pathway in response to osmotic stress [GO:1902219]; positively regulated by GO:1902220